regulation of miRNA-mediated gene silencing [GO:0060964] (biological process) Also known as: regulation of gene silencing by miRNA, regulation of gene silencing by microRNA References: PMID:23985560, PMID:28379604 Sources: GOC:aruk, GOC:bc, GOC:dph, GOC:rl, GOC:tb Relationships: is a type of regulation of post-transcriptional gene silencing by regulatory ncRNA [GO:1900368]; regulates miRNA-mediated post-transcriptional gene silencing [GO:0035195] Subtypes: negative regulation of miRNA-mediated gene silencing [GO:0060965], positive regulation of miRNA-mediated gene silencing [GO:2000637] Definition: A process that modulates the rate, frequency, or extent of the downregulation of gene expression through the action of microRNAs (miRNAs).